{
  "term_label": "adenylate cyclase-activating G protein-coupled receptor signaling pathway",
  "gene_symbol": "PRKAR2A",
  "gene_name": "cAMP-dependent protein kinase type II-alpha regulatory subunit",
  "term_id": "GO:0007189",
  "gene": "UniProtKB:P13861"
}